{
  "gene_symbol": "IFT20",
  "gene": "UniProtKB:Q8IY31",
  "gene_name": "Intraflagellar transport protein 20 homolog",
  "term_label": "ciliary basal body",
  "term_id": "GO:0036064"
}